{
  "term_label": "Unknown molecular function",
  "gene_name": "Interactor of HORMAD1 protein 1",
  "gene": "UniProtKB:Q8IYA8",
  "term_id": "UNKNOWN:0001",
  "gene_symbol": "IHO1"
}